{
  "term_label": "DNA-binding transcription factor activity, RNA polymerase II-specific",
  "gene_symbol": "ZNF470",
  "gene": "UniProtKB:Q6ECI4",
  "term_id": "GO:0000981",
  "gene_name": "Zinc finger protein 470"
}